perillyl-alcohol dehydrogenase (NAD+) activity [GO:0018457] (molecular function) Sources: EC:1.1.1.144, RHEA:10664 Definition: Catalysis of the reaction: NAD+ + perillyl alcohol = H+ + NADH + perillyl aldehyde. Also known as: perillyl-alcohol dehydrogenase activity, perillyl alcohol dehydrogenase activity, perillyl-alcohol:NAD+ oxidoreductase activity Relationships: is a type of alcohol dehydrogenase (NAD+) activity [GO:0004022]